{
  "gene_symbol": "ERF",
  "term_id": "GO:0005634",
  "gene_name": "ETS domain-containing transcription factor ERF",
  "term_label": "nucleus",
  "gene": "UniProtKB:P50548"
}